positive regulation of insulin receptor signaling pathway [GO:0046628] (biological process) Sources: GOC:bf Definition: Any process that increases the frequency, rate or extent of insulin receptor signaling. Relationships: is a type of positive regulation of signal transduction [GO:0009967]; is a type of regulation of insulin receptor signaling pathway [GO:0046626]; is a type of GO:1900078; positively regulates GO:0008286 Also known as: positive regulation of insulin receptor signalling pathway, up regulation of insulin receptor signaling pathway, up-regulation of insulin receptor signaling pathway, upregulation of insulin receptor signaling pathway, activation of insulin receptor signaling pathway, stimulation of insulin receptor signaling pathway Subtypes: positive regulation of insulin receptor signaling pathway by insulin receptor internalization [GO:0038015]